{
  "term_label": "positive regulation of type 2 immune response",
  "gene_symbol": "CD74",
  "term_id": "GO:0002830",
  "gene_name": "HLA class II histocompatibility antigen gamma chain",
  "gene": "UniProtKB:P04233"
}